{
  "gene": "UniProtKB:Q13503",
  "term_label": "regulation of transcription by RNA polymerase II",
  "gene_symbol": "MED21",
  "term_id": "GO:0006357",
  "gene_name": "Mediator of RNA polymerase II transcription subunit 21"
}